{
  "gene": "UniProtKB:Q9NVC3",
  "gene_name": "Sodium-coupled neutral amino acid transporter 7",
  "term_label": "amino acid transmembrane transport",
  "gene_symbol": "SLC38A7",
  "term_id": "GO:0003333"
}